neural rod formation [GO:0014023] (biological process) Relationships: is a type of anatomical structure formation involved in morphogenesis [GO:0048646]; is part of primary neural tube formation [GO:0014020] Sources: GOC:dh, GOC:ef Definition: The formation of a solid rod of neurectoderm derived from the neural keel. The neural rod is roughly circular in cross section. Neural rod formation occurs during primary neurulation in teleosts.